{
  "term_label": "mitochondrion",
  "gene_name": "Inorganic pyrophosphatase 2, mitochondrial",
  "term_id": "GO:0005739",
  "gene": "UniProtKB:Q9H2U2",
  "gene_symbol": "PPA2"
}